XCR1 chemokine receptor binding [GO:0031738] (molecular function) Sources: GOC:mah, GOC:nln Definition: Binding to a XCR1 chemokine receptor. Relationships: is a type of chemokine receptor binding [GO:0042379] Also known as: lymphotactin receptor binding, XCR1 chemokine receptor ligand